melanotic encapsulation of foreign target [GO:0035011] (biological process) Regulation: regulated by regulation of melanotic encapsulation of foreign target [GO:0140539]; negatively regulated by negative regulation melanotic encapsulation of foreign target [GO:0140540] Relationships: is a type of melanization defense response [GO:0035006]; is a type of encapsulation of foreign target [GO:0035010] Sources: GOC:bf Definition: Formation of a multilayered, melanized sheath of cells around a foreign invader.